G protein-coupled peptide receptor activity [GO:0008528] (molecular function) Definition: Combining with a peptide and transmitting the signal across the membrane by activating an associated G-protein; promotes the exchange of GDP for GTP on the alpha subunit of a heterotrimeric G-protein complex. Sources: GOC:dph, GOC:tb Also known as: G protein coupled peptide receptor activity, G-protein coupled peptide receptor activity, peptide receptor activity, G protein coupled, peptide receptor activity, G-protein coupled Relationships: is a type of GO:0001653; is a type of GO:0004930 Subtypes: angiotensin receptor activity [GO:0001595], urotensin II receptor activity [GO:0001604], nociceptin receptor activity [GO:0001626], proteinase-activated receptor activity [GO:0001648], GO:0004932, bradykinin receptor activity [GO:0004947], cholecystokinin receptor activity [GO:0004951], endothelin receptor activity [GO:0004962], glucagon receptor activity [GO:0004967], melanocortin receptor activity [GO:0004977], N-formyl peptide receptor activity [GO:0004982], oxytocin receptor activity [GO:0004990], vasopressin receptor activity [GO:0005000], GO:0008188, allatostatin receptor activity [GO:0008261], gastrin receptor activity [GO:0015054], orexin receptor activity [GO:0016499], myosuppressin receptor activity [GO:0035013], GO:0036318, G protein-coupled enkephalin receptor activity [GO:0038046], GO:0038048, GO:0044508, GO:0060182, GO:0097642